{
  "term_label": "G protein-coupled receptor activity",
  "term_id": "GO:0004930",
  "gene_name": "Mas-related G-protein coupled receptor member F",
  "gene": "UniProtKB:Q96AM1",
  "gene_symbol": "MRGPRF"
}